{
  "gene_name": "Neuronal PAS domain-containing protein 3",
  "gene": "UniProtKB:Q8IXF0",
  "gene_symbol": "NPAS3",
  "term_label": "nucleus",
  "term_id": "GO:0005634"
}